{
  "gene_symbol": "ANGPT2",
  "term_label": "angiogenesis",
  "gene_name": "Angiopoietin-2",
  "gene": "UniProtKB:O15123",
  "term_id": "GO:0001525"
}